core mediator complex [GO:0070847] (cellular component) Also known as: C mediator complex, S mediator complex Relationships: is a type of RNA polymerase II transcription regulator complex [GO:0090575] References: PMID:11454195, PMID:16168358, PMID:17870225 Definition: A protein complex that interacts with the carboxy-terminal domain of the largest subunit of RNA polymerase II and plays an active role in transducing the signal from a transcription factor to the transcriptional machinery. The core mediator complex has a stimulatory effect on basal transcription, and contains most of the same subdomains as the larger form of mediator complex -- a head domain comprising proteins known in Saccharomyces as Srb2, -4, and -5, Med6, -8, and -11, and Rox3 proteins; a middle domain comprising Med1, -4, and -7, Nut1 and -2, Cse2, Rgr1, Soh1, and Srb7 proteins; and a tail consisting of Gal11p, Med2p, Pgd1p, and Sin4p -- but lacks the regulatory subcomplex comprising Ssn2, -3, and -8, and Srb8 proteins. Metazoan core mediator complexes have similar modular structures and include homologs of yeast Srb and Med proteins.